{
  "term_id": "UNKNOWN:0002",
  "gene": "UniProtKB:Q9UK28",
  "gene_symbol": "TMEM59L",
  "gene_name": "Transmembrane protein 59-like",
  "term_label": "Unknown biological process"
}